{
  "term_id": "GO:0000981",
  "gene_symbol": "LHX9",
  "gene": "UniProtKB:Q9NQ69",
  "term_label": "DNA-binding transcription factor activity, RNA polymerase II-specific",
  "gene_name": "LIM_homeobox protein Lhx9"
}